{
  "term_id": "GO:0000981",
  "gene": "UniProtKB:Q9H2C1",
  "term_label": "DNA-binding transcription factor activity, RNA polymerase II-specific",
  "gene_symbol": "LHX5",
  "gene_name": "LIM_homeobox protein Lhx5"
}